{
  "gene_symbol": "PNMA8B",
  "gene": "UniProtKB:Q9ULN7",
  "term_id": "UNKNOWN:0001",
  "term_label": "Unknown molecular function",
  "gene_name": "Paraneoplastic antigen-like protein 8B"
}